positive regulation of growth plate cartilage chondrocyte proliferation [GO:0061913] (BP) References: PMID:19264869 Definition: Any process that increases the rate, frequency, or extent of the multiplication or reproduction of chondrocytes in a growing endochondral bone, resulting in the expansion of a cell population. Relationships: is a type of regulation of growth plate cartilage chondrocyte proliferation [GO:0003420]; is_a positive regulation of cell population proliferation [GO:0008284]; positively regulates growth plate cartilage chondrocyte proliferation [GO:0003419]